{
  "term_id": "UNKNOWN:0003",
  "gene_symbol": "FAM163A",
  "term_label": "Unknown cellular component",
  "gene_name": "Protein FAM163A",
  "gene": "UniProtKB:Q96GL9"
}